gamma-aminobutyric acid transmembrane transporter activity [GO:0015185] (molecular function) Also known as: 4-aminobutanoate transporter activity, 4-aminobutyrate transporter activity, GABA transporter activity, betaine/GABA:sodium symporter activity Relationships: is a type of GO:0008028; is a type of amino acid transmembrane transporter activity [GO:0015171]; is part of GO:0015812 Sources: GOC:go_curators, GOC:mtg_transport, ISBN:0198506732, ISBN:0815340729 Definition: Enables the transfer of gamma-aminobutyric acid from one side of a membrane to the other. Gamma-aminobutyric acid is 4-aminobutyrate (GABA). Subtypes: gamma-aminobutyric acid:sodium:chloride symporter activity [GO:0005332], gamma-aminobutyric acid:proton symporter activity [GO:0015495], GO:0070909, gamma-aminobutyric acid:proton antiporter activity [GO:0140800]